peptidoglycan asparagine synthase activity [GO:0102115] (molecular function) Definition: Catalysis of the reaction: ditrans,octacis-undecaprenyldiphospho-N-acetyl-(N-acetylglucosaminyl)muramoyl-L-alanyl-gamma-D-isoglutaminyl-N-(beta-D-asparatyl)-L-lysyl-D-alanyl-D-alanine + ammonium + ATP = H+ + ditrans,octacis-undecaprenyldiphospho-N-acetyl-(N-acetylglucosaminyl)muramoyl-L-alanyl-gamma-D-isoglutaminyl-N-(beta-D-asparaginyl)-L-lysyl-D-alanyl-D-alanine + AMP + diphosphoric acid. Sources: EC:6.3.1.-, GOC:pz Relationships: is a type of GO:0016880